{
  "term_id": "UNKNOWN:0002",
  "gene_name": "Large ribosomal subunit protein mL39",
  "gene": "UniProtKB:Q9NYK5",
  "term_label": "Unknown biological process",
  "gene_symbol": "MRPL39"
}